{
  "gene": "UniProtKB:Q96P63",
  "gene_symbol": "SERPINB12",
  "term_label": "extracellular space",
  "gene_name": "Serpin B12",
  "term_id": "GO:0005615"
}